{
  "term_label": "defense response",
  "gene_symbol": "NOX5",
  "term_id": "GO:0006952",
  "gene": "UniProtKB:Q96PH1",
  "gene_name": "NADPH oxidase 5"
}